{
  "gene_name": "Enoyl-CoA delta isomerase 2",
  "gene_symbol": "ECI2",
  "term_label": "fatty acid beta-oxidation",
  "gene": "UniProtKB:O75521",
  "term_id": "GO:0006635"
}